T=pseudo3 icosahedral viral capsid [GO:0039618] (cellular component) Note: T=pseudo3 capsids are not T=3 symmetry as described by Caspar and Klug (PMID:14019094) because the basic unit is composed of three different proteins. Since the three subunits are morphologically very similar, the structure is therefore a pseudo T=3. Relationships: is a type of icosahedral viral capsid [GO:0019030] Sources: VZ:809 Definition: The protein coat that surrounds the infective nucleic acid in some virus particles where the subunits (capsomeres) are arranged to form an icosahedron with pseudo T=3 symmetry. The T=pseudo3 capsid is composed of 12 pentameric and 20 hexameric capsomeres.